mitotic spindle disassembly [GO:0051228] (biological process) Regulation: regulated by regulation of mitotic spindle disassembly [GO:1904686]; positively regulated by positive regulation of mitotic spindle disassembly [GO:1904687] Sources: GOC:ai Also known as: mitotic spindle breakdown, mitotic spindle catabolism, mitotic spindle degradation, spindle breakdown during mitosis, spindle degradation during mitosis, spindle disassembly during mitosis Relationships: is a type of mitotic spindle organization [GO:0007052]; is a type of GO:0051230 Definition: The controlled breakdown of the spindle during a mitotic cell cycle.